{
  "term_id": "GO:0005829",
  "term_label": "cytosol",
  "gene": "UniProtKB:Q16772",
  "gene_name": "Glutathione S-transferase A3",
  "gene_symbol": "GSTA3"
}